S-alkylthiohydroximate lyase activity [GO:0080108] (molecular function) Relationships: is a type of GO:0016846 References: PMID:14871316 Also known as: S-alkylthiohydroximate C-S lyase activity Definition: Catalysis of the conversion of a S-alkylthiohydroximate to a thiohydroximate.